immunoglobulin receptor activity [GO:0019763] (molecular function) Definition: Combining with the Fc region of an immunoglobulin protein and transmitting the signal from one side of the membrane to the other to initiate a change in cell activity. Subtypes: polymeric immunoglobulin receptor activity [GO:0001792], IgM receptor activity [GO:0001793], IgA receptor activity [GO:0019766], GO:0019767, GO:0019770 Relationships: is a type of transmembrane signaling receptor activity [GO:0004888]; is a type of immune receptor activity [GO:0140375]; BFO_0000050 Fc receptor signaling pathway [GO:0038093]; BFO_0000051 GO:0019865 Also known as: FC receptor activity Sources: GOC:signaling, ISBN:0198547684